{
  "gene": "UniProtKB:P01189",
  "gene_symbol": "POMC",
  "gene_name": "Pro-opiomelanocortin",
  "term_label": "secretory granule",
  "term_id": "GO:0030141"
}